transcription repressor complex [GO:0017053] (CC) Sources: GOC:mah Also known as: transcription factor inhibitor complex, transcriptional repressor complex, cytoplasmic transcriptional repressor complex, nuclear transcriptional repressor complex Relationships: is a type of transcription regulator complex [GO:0005667] Definition: A protein complex that possesses activity that prevents or downregulates transcription. Subtypes: H-NS-Cnu complex [GO:0036411], GO:0090570, RNA polymerase II transcription repressor complex [GO:0090571], RNA polymerase III transcription repressor complex [GO:0090572], RNA polymerase IV transcription repressor complex [GO:0090573], RNA polymerase V transcription repressor complex [GO:0090574], GO:0110001, Cry-Per complex [GO:1990512]